{
  "gene_name": "5-hydroxytryptamine receptor 1A",
  "gene_symbol": "HTR1A",
  "term_id": "GO:0007187",
  "term_label": "G protein-coupled receptor signaling pathway, coupled to cyclic nucleotide second messenger",
  "gene": "UniProtKB:P08908"
}